{
  "term_id": "GO:0002142",
  "gene_symbol": "USH1C",
  "gene_name": "Harmonin",
  "term_label": "stereocilia ankle link complex",
  "gene": "UniProtKB:Q9Y6N9"
}